embryonic placenta development [GO:0001892] (biological process) Definition: The embryonically driven process whose specific outcome is the progression of the placenta over time, from its formation to the mature structure. The placenta is an organ of metabolic interchange between fetus and mother, partly of embryonic origin and partly of maternal origin. Sources: GOC:add, ISBN:068340007X Also known as: fetal placenta development Relationships: is a type of embryonic organ development [GO:0048568]; is part of GO:0001701; is part of placenta development [GO:0001890]